ubiquitin-specific protease binding [GO:1990381] (molecular function) References: PMID:24063750 Sources: GOC:PARL, GOC:bf Relationships: is a type of GO:0002020 Also known as: deubiquitinase binding, deubiquitinating enzyme binding Definition: Binding to a ubiquitin-specific protease.